amnioserosa maintenance [GO:0046665] (biological process) Relationships: is a type of GO:0001894; is part of embryonic development via the syncytial blastoderm [GO:0001700] Sources: GOC:bf Definition: Maintenance of the amnioserosa, an epithelium that occupies a hole in the embryonic dorsal epidermis.